{
  "gene_name": "Neuropeptide S receptor",
  "term_label": "plasma membrane",
  "gene_symbol": "NPSR1",
  "gene": "UniProtKB:Q6W5P4",
  "term_id": "GO:0005886"
}